{
  "gene": "UniProtKB:P78333",
  "term_id": "UNKNOWN:0001",
  "term_label": "Unknown molecular function",
  "gene_name": "Glypican-5",
  "gene_symbol": "GPC5"
}